tripartite attachment complex [GO:0120121] (cellular component) Also known as: TAC Definition: A three-part cytoskeletal structure in kinetoplastid species linking mitochondrial DNA organised in a kinetoplast through the mitochondrial membranes to the basal body. Relationships: is a type of cellular anatomical structure [GO:0110165]; is part of cytoskeleton [GO:0005856] References: PMID:12802053, PMID:18059470, PMID:24821793, PMID:27168148